zinc:bicarbonate symporter activity [GO:0140412] (molecular function) Subtypes: zinc:bicarbonate:selenite symporter activity [GO:0140413] Also known as: zinc:hydrogencarbonate symporter activity References: PMID:27166256 Definition: Enables the transfer of a solute or solutes from one side of a membrane to the other according to the reaction: zinc(out) + HCO3-(out) = zinc(in) + HCO3-(in). Relationships: is a type of zinc ion transmembrane transporter activity [GO:0005385]; is a type of GO:0140410